agmatine N4-coumaroyltransferase activity [GO:0047634] (molecular function) Also known as: 4-coumaroyl-CoA:agmatine 4-N-coumaroyltransferase activity, 4-coumaroyl-CoA:agmatine N4-coumaroyltransferase activity, agmatine coumaroyltransferase activity, p-coumaroyl-CoA-agmatine N-p-coumaroyltransferase activity Relationships: is a type of GO:0016747 Definition: Catalysis of the reaction: 4-coumaroyl-CoA + agmatine = N-(4-guanidiniumylbutyl)-4-hydroxycinnamamide + CoA + H+. Sources: EC:2.3.1.64, RHEA:13405